{
  "gene_symbol": "CYP51A1",
  "term_id": "GO:0033488",
  "term_label": "cholesterol biosynthetic process via 24,25-dihydrolanosterol",
  "gene": "UniProtKB:Q16850",
  "gene_name": "Lanosterol 14-alpha demethylase"
}